{
  "gene_name": "Sodium_hydrogen exchanger 6",
  "term_id": "GO:0015385",
  "gene": "UniProtKB:Q92581",
  "term_label": "sodium:proton antiporter activity",
  "gene_symbol": "SLC9A6"
}